{
  "gene_symbol": "TRPM5",
  "gene": "UniProtKB:Q9NZQ8",
  "gene_name": "Transient receptor potential cation channel subfamily M member 5",
  "term_label": "plasma membrane",
  "term_id": "GO:0005886"
}